{
  "gene_name": "Prokineticin-1",
  "term_label": "Unknown cellular component",
  "term_id": "UNKNOWN:0003",
  "gene": "UniProtKB:P58294",
  "gene_symbol": "PROK1"
}